{
  "term_id": "GO:0005634",
  "gene": "UniProtKB:Q16385",
  "term_label": "nucleus",
  "gene_symbol": "SSX2B",
  "gene_name": "Protein SSX2"
}